{
  "gene_symbol": "AGO3",
  "gene": "UniProtKB:Q9H9G7",
  "gene_name": "Protein argonaute-3",
  "term_id": "GO:0005634",
  "term_label": "nucleus"
}